{
  "term_label": "olfactory receptor activity",
  "gene_name": "Olfactory receptor 2T12",
  "term_id": "GO:0004984",
  "gene_symbol": "OR2T12",
  "gene": "UniProtKB:Q8NG77"
}